piP-body [GO:0071547] (cellular component) Definition: A P granule that contains the PIWIL4-TDRD9 module, a set of proteins that act in the secondary piRNA pathway. References: PMID:20011505 Sources: GOC:sp Relationships: is a type of P granule [GO:0043186]